{
  "term_id": "GO:0006368",
  "gene_name": "RNA polymerase-associated protein CTR9 homolog",
  "gene_symbol": "CTR9",
  "gene": "UniProtKB:Q6PD62",
  "term_label": "transcription elongation by RNA polymerase II"
}